neosartoricin biosynthetic process [GO:1902050] (biological process) Also known as: neosartoricin anabolism, neosartoricin biosynthesis, neosartoricin formation, neosartoricin synthesis Regulation: regulated by regulation of neosartoricin biosynthetic process [GO:1902053]; negatively regulated by negative regulation of neosartoricin biosynthetic process [GO:1902054]; positively regulated by positive regulation of neosartoricin biosynthetic process [GO:1902055] Relationships: is a type of GO:0030639; is a type of ketone biosynthetic process [GO:0042181]; is a type of phenol-containing compound biosynthetic process [GO:0046189]; is a type of GO:1902645 Definition: The chemical reactions and pathways resulting in the formation of neosartoricin. References: PMID:23368997 Sources: GOC:TermGenie, GOC:di